{
  "term_id": "GO:0005737",
  "gene": "UniProtKB:Q14681",
  "gene_name": "BTB_POZ domain-containing protein KCTD2",
  "term_label": "cytoplasm",
  "gene_symbol": "KCTD2"
}